{
  "gene": "UniProtKB:Q13018",
  "gene_symbol": "PLA2R1",
  "term_id": "GO:0006898",
  "term_label": "receptor-mediated endocytosis",
  "gene_name": "Secretory phospholipase A2 receptor"
}